{
  "term_id": "GO:0005789",
  "gene_name": "Rhomboid domain-containing protein 2",
  "term_label": "endoplasmic reticulum membrane",
  "gene_symbol": "RHBDD2",
  "gene": "UniProtKB:Q6NTF9"
}